{
  "gene": "UniProtKB:Q9Y6Z2",
  "term_id": "UNKNOWN:0003",
  "gene_name": "Uncharacterized protein encoded by LINC01558",
  "term_label": "Unknown cellular component",
  "gene_symbol": "LINC01558"
}